{
  "gene": "UniProtKB:Q96MV8",
  "gene_name": "Palmitoyltransferase ZDHHC15",
  "gene_symbol": "ZDHHC15",
  "term_label": "endoplasmic reticulum",
  "term_id": "GO:0005783"
}